{
  "gene": "UniProtKB:Q9C0D6",
  "term_id": "GO:0030041",
  "gene_name": "FH2 domain-containing protein 1",
  "term_label": "actin filament polymerization",
  "gene_symbol": "FHDC1"
}